{
  "gene": "UniProtKB:Q8NFZ8",
  "gene_name": "Cell adhesion molecule 4",
  "gene_symbol": "CADM4",
  "term_id": "GO:0044291",
  "term_label": "cell-cell contact zone"
}